nonadec-1-ene biosynthetic process [GO:1900877] (biological process) Relationships: is a type of alkene biosynthetic process [GO:0043450]; is a type of GO:1900876 Regulation: RO_0002211 by GO:1900935; negatively regulated by negative regulation of nonadec-1-ene biosynthetic process [GO:1900936]; positively regulated by positive regulation of nonadec-1-ene biosynthetic process [GO:1900937] Also known as: nonadec-1-ene anabolism, nonadec-1-ene biosynthesis, nonadec-1-ene formation, nonadec-1-ene synthesis Sources: GOC:TermGenie, GOC:mengo_curators Definition: The chemical reactions and pathways resulting in the formation of nonadec-1-ene.